{
  "gene_name": "Sodium- and chloride-dependent glycine transporter 1",
  "gene": "UniProtKB:P48067",
  "gene_symbol": "SLC6A9",
  "term_id": "GO:1903804",
  "term_label": "glycine import across plasma membrane"
}